{
  "term_id": "UNKNOWN:0003",
  "gene": "UniProtKB:Q9BTE3",
  "gene_symbol": "MCMBP",
  "gene_name": "Mini-chromosome maintenance complex-binding protein",
  "term_label": "Unknown cellular component"
}